{
  "term_id": "GO:0003723",
  "gene_symbol": "CAPRIN1",
  "term_label": "RNA binding",
  "gene_name": "Caprin-1",
  "gene": "UniProtKB:Q14444"
}